{
  "term_id": "GO:0006412",
  "gene_name": "Large ribosomal subunit protein bL12m",
  "gene_symbol": "MRPL12",
  "term_label": "translation",
  "gene": "UniProtKB:P52815"
}